{
  "term_label": "Unknown molecular function",
  "gene": "UniProtKB:Q5T440",
  "gene_name": "Putative transferase CAF17, mitochondrial",
  "gene_symbol": "IBA57",
  "term_id": "UNKNOWN:0001"
}